9,12-octadecadienoate 8-hydroperoxide 8S-isomerase activity [GO:0052879] (molecular function) Definition: Catalysis of the reaction: (8R,9Z,12Z)-8-hydroperoxyoctadeca-9,12-dienoate = (7S,8S,9Z,12Z)-7,8-dihydroxyoctadeca-9,12-dienoate. Sources: RHEA:25399 Also known as: 8-hydroperoxide isomerase activity, (8R,9Z,12Z)-8-hydroperoxy-9,12-octadecadienoate mutase ((7S,8S,9Z,12Z)-5,8-dihydroxy-9,12-octadecadienoate-forming) activity, linoleate diol synthase activity Relationships: is a type of GO:0050486